{
  "gene_name": "17-beta-hydroxysteroid dehydrogenase type 2",
  "term_id": "GO:0004303",
  "gene": "UniProtKB:P37059",
  "gene_symbol": "HSD17B2",
  "term_label": "estradiol 17-beta-dehydrogenase [NAD(P)+] activity"
}